heart valve cell differentiation [GO:0003293] (biological process) Definition: The process in which an endocardial cushion cell give rise to a cell that is part of a heart valve. Relationships: is_a cardiocyte differentiation [GO:0035051]; is part of heart valve development [GO:0003170] Sources: GOC:mtg_heart